{
  "gene": "UniProtKB:Q8N6F1",
  "gene_name": "Claudin-19",
  "gene_symbol": "CLDN19",
  "term_id": "GO:0160184",
  "term_label": "paracellular transport"
}